{
  "term_label": "cristae formation",
  "term_id": "GO:0042407",
  "gene_name": "MICOS complex subunit MIC60",
  "gene": "UniProtKB:Q16891",
  "gene_symbol": "IMMT"
}